(R)-mandelate catabolic process to benzoate [GO:0019597] (biological process) Sources: GOC:go_curators Also known as: (R)-mandelate breakdown to benzoate, (R)-mandelate degradation to benzoate Definition: The chemical reactions and pathways resulting in the breakdown of (R)-mandelate into other compounds, including benzoate. Relationships: is a type of benzoate metabolic process [GO:0018874]; is a type of mandelate catabolic process [GO:0019596]; is a type of monocarboxylic acid biosynthetic process [GO:0072330]